isochorismatase activity [GO:0008908] (molecular function) Relationships: is a type of leukotriene-A4 hydrolase activity [GO:0004463] Also known as: 2,3 dihydro-2,3 dihydroxybenzoate synthase activity, 2,3-dihydro-2,3-dihydroxybenzoate synthase activity, 2,3-dihydroxy-2,3-dihydrobenzoate synthase activity, 2,3-dihydroxy-2,3-dihydrobenzoic synthase activity, isochorismate pyruvate-hydrolase activity Sources: EC:3.3.2.1, RHEA:11112 Definition: Catalysis of the reaction: H2O + isochorismate = 2,3-dihydroxy-2,3-dihydrobenzoate + pyruvate.